nucleoside catabolic process [GO:0009164] (biological process) Definition: The chemical reactions and pathways resulting in the breakdown of any one of a family of organic molecules consisting of a purine or pyrimidine base covalently bonded to a sugar ribose (a ribonucleoside) or deoxyribose (a deoxyribonucleoside). Sources: GOC:jl Relationships: is_a nucleoside metabolic process [GO:0009116]; is a type of nucleobase-containing small molecule catabolic process [GO:0034656]; is a type of glycosyl compound catabolic process [GO:1901658] Also known as: nucleoside breakdown, nucleoside catabolism, nucleoside degradation Subtypes: purine nucleoside catabolic process [GO:0006152], ribonucleoside catabolic process [GO:0042454], deoxyribonucleoside catabolic process [GO:0046121], pyrimidine nucleoside catabolic process [GO:0046135], pyridine nucleoside catabolic process [GO:0070638]